{
  "gene": "UniProtKB:O95025",
  "gene_symbol": "SEMA3D",
  "term_label": "extracellular space",
  "term_id": "GO:0005615",
  "gene_name": "Semaphorin-3D"
}